collagen type XXVI trimer [GO:1990324] (cellular component) Definition: A collagen homotrimer of alpha1(XXVI) chains. Relationships: is a type of collagen trimer [GO:0005581]; is part of GO:0140152 References: PMID:17876790 Sources: GOC:bhm